{
  "term_label": "nucleus",
  "gene_name": "Aprataxin and PNK-like factor",
  "term_id": "GO:0005634",
  "gene": "UniProtKB:Q8IW19",
  "gene_symbol": "APLF"
}